ER retention sequence binding [GO:0046923] (molecular function) Subtypes: KDEL sequence binding [GO:0005046], DDEL sequence binding [GO:0030944], HDEL sequence binding [GO:0045015] Definition: Binding to an endoplasmic reticulum (ER) retention sequence, a specific peptide sequence that ensures a protein is retained within the ER. Relationships: is a type of signal sequence binding [GO:0005048] Sources: GOC:ai Also known as: endoplasmic reticulum retention sequence binding